{
  "gene_name": "WD repeat and FYVE domain-containing protein 2",
  "term_id": "GO:0005769",
  "term_label": "early endosome",
  "gene": "UniProtKB:Q96P53",
  "gene_symbol": "WDFY2"
}